{
  "gene": "UniProtKB:P31943",
  "gene_name": "Heterogeneous nuclear ribonucleoprotein H",
  "term_label": "RNA binding",
  "gene_symbol": "HNRNPH1",
  "term_id": "GO:0003723"
}